immune system development [GO:0002520] (biological process) Definition: The process whose specific outcome is the progression of an organismal system whose objective is to provide calibrated responses by an organism to a potential internal or invasive threat, over time, from its formation to the mature structure. A system is a regularly interacting or interdependent group of organs or tissues that work together to carry out a given biological process. Sources: GOC:add, GOC:dph Relationships: is a type of immune system process [GO:0002376]; is a type of system development [GO:0048731]